{
  "gene": "UniProtKB:Q9P2S2",
  "gene_symbol": "NRXN2",
  "gene_name": "Neurexin-2",
  "term_label": "nervous system development",
  "term_id": "GO:0007399"
}